inositol-1-diphosphate-2,3,4,5,6-pentakisphosphate diphosphatase activity [GO:0052843] (molecular function) References: PMID:10827188, PMID:11502751, PMID:26422458 Definition: Catalysis of the reaction: 1-diphospho-1D-myo-inositol 2,3,4,5,6-pentakisphosphate + H2O = 1D-myo-inositol 1,2,3,4,5,6-hexakisphosphate + phosphate + 2 H+. Relationships: is a type of inositol diphosphate pentakisphosphate diphosphatase activity [GO:0052842] Also known as: inositol 1-diphosphate 2,3,4,5,6-pentakisphosphate 1-diphosphatase activity, inositol 1-pyrophosphate 2,3,4,5,6-pentakisphosphate 1-pyrophosphatase activity